{
  "term_id": "GO:0097352",
  "gene": "UniProtKB:Q9H714",
  "term_label": "autophagosome maturation",
  "gene_symbol": "RUBCNL",
  "gene_name": "Protein associated with UVRAG as autophagy enhancer"
}